{
  "gene_name": "T cell receptor alpha joining 24 (Fragment)",
  "gene_symbol": "TRAJ24",
  "term_id": "UNKNOWN:0003",
  "term_label": "Unknown cellular component",
  "gene": "UniProtKB:A0A075B6Z9"
}